{
  "gene_symbol": "NECTIN2",
  "gene_name": "Nectin-2",
  "gene": "UniProtKB:Q92692",
  "term_label": "homophilic cell-cell adhesion",
  "term_id": "GO:0007156"
}